{
  "term_label": "Unknown cellular component",
  "gene_name": "E3 ubiquitin-protein ligase TRIM8",
  "gene_symbol": "TRIM8",
  "gene": "UniProtKB:Q9BZR9",
  "term_id": "UNKNOWN:0003"
}